{
  "term_label": "epidermis development",
  "term_id": "GO:0008544",
  "gene": "UniProtKB:A6NHS7",
  "gene_symbol": "MANSC4",
  "gene_name": "MANSC domain-containing protein 4"
}